{
  "gene_symbol": "BEND3",
  "gene": "UniProtKB:Q5T5X7",
  "term_id": "GO:0000182",
  "term_label": "rDNA binding",
  "gene_name": "BEN domain-containing protein 3"
}